{
  "gene_name": "Roquin-1",
  "gene": "UniProtKB:Q5TC82",
  "gene_symbol": "RC3H1",
  "term_label": "protein polyubiquitination",
  "term_id": "GO:0000209"
}